{
  "gene": "UniProtKB:P40123",
  "term_id": "GO:0003779",
  "gene_symbol": "CAP2",
  "term_label": "actin binding",
  "gene_name": "Adenylyl cyclase-associated protein 2"
}